chromatin-protein adaptor activity [GO:0140463] (molecular function) References: PMID:32277274 Relationships: is a type of protein-macromolecule adaptor activity [GO:0030674]; is part of GO:0006325; has part chromatin binding [GO:0003682] Also known as: chromatin adaptor, chromatin adaptor activity, chromatin receptor, chromatin-protein adaptor, protein-chromatin adaptor activity, chromatin recruitment Subtypes: histone reader activity [GO:0140566], dsDNA-RNA triple helix-forming chromatin adaptor activity [GO:0141180] Definition: An adaptor activity that brings together a protein and a region of the chromatin, such as a nucleosome, to establish or maintain the chromatin localization of the protein, or the complex to which it belongs.